calcium ion-transporting ATPase complex [GO:0090534] (CC) Definition: Protein complex that carries out the reaction: ATP + H2O + Ca2+(out) = ADP + phosphate + Ca2+(in). Relationships: is a type of cation-transporting ATPase complex [GO:0090533] Sources: GOC:BHF